{
  "gene_symbol": "ZNF619",
  "term_label": "regulation of transcription by RNA polymerase II",
  "gene_name": "Zinc finger protein 619",
  "gene": "UniProtKB:Q8N2I2",
  "term_id": "GO:0006357"
}